{
  "gene": "UniProtKB:Q8N1D0",
  "gene_name": "Beckwith-Wiedemann syndrome chromosomal region 1 candidate gene B protein",
  "gene_symbol": "SLC22A18AS",
  "term_id": "UNKNOWN:0003",
  "term_label": "Unknown cellular component"
}